{
  "gene": "UniProtKB:Q9BYR0",
  "gene_name": "Keratin-associated protein 4-7",
  "gene_symbol": "KRTAP4-7",
  "term_label": "hair cycle",
  "term_id": "GO:0042633"
}